alpha-ribazole phosphatase activity [GO:0043755] (MF) Definition: Catalysis of the reaction: alpha-ribazole 5'-phosphate + H2O = alpha-ribazole + phosphate. Sources: RHEA:24456 Also known as: alpha-ribazole-5'-P phosphatase activity, alpha-ribazole-5'-phosphate phosphohydrolase activity, CobC Relationships: is a type of GO:0016791